{
  "gene": "UniProtKB:Q9H8M9",
  "term_id": "UNKNOWN:0001",
  "term_label": "Unknown molecular function",
  "gene_symbol": "EVA1A",
  "gene_name": "Protein eva-1 homolog A"
}